{
  "gene": "UniProtKB:O60936",
  "gene_name": "Nucleolar protein 3",
  "term_label": "negative regulation of extrinsic apoptotic signaling pathway",
  "gene_symbol": "NOL3",
  "term_id": "GO:2001237"
}